{
  "gene": "UniProtKB:Q9Y371",
  "term_label": "membrane",
  "gene_symbol": "SH3GLB1",
  "gene_name": "Endophilin-B1",
  "term_id": "GO:0016020"
}